{
  "term_id": "UNKNOWN:0002",
  "gene": "UniProtKB:O00212",
  "term_label": "Unknown biological process",
  "gene_symbol": "RHOD",
  "gene_name": "Rho-related GTP-binding protein RhoD"
}